{
  "gene_symbol": "RPUSD2",
  "gene": "UniProtKB:Q8IZ73",
  "gene_name": "Pseudouridylate synthase RPUSD2",
  "term_id": "GO:0000455",
  "term_label": "enzyme-directed rRNA pseudouridine synthesis"
}